{
  "gene": "UniProtKB:Q12802",
  "term_id": "GO:0043410",
  "gene_symbol": "AKAP13",
  "gene_name": "A-kinase anchor protein 13",
  "term_label": "positive regulation of MAPK cascade"
}